{
  "term_id": "GO:0016020",
  "gene_symbol": "BBS7",
  "gene_name": "Bardet-Biedl syndrome 7 protein",
  "term_label": "membrane",
  "gene": "UniProtKB:Q8IWZ6"
}